regulation of establishment of protein localization [GO:0070201] (biological process) Also known as: regulation of establishment of protein localisation Definition: Any process that modulates the frequency, rate or extent of the directed movement of a protein to a specific location. Subtypes: regulation of protein transport [GO:0051223], GO:0070202, regulation of protein targeting [GO:1903533], regulation of establishment of protein localization to mitochondrion [GO:1903747], negative regulation of establishment of protein localization [GO:1904950], GO:1904951 Relationships: is_a regulation of protein localization [GO:0032880]; regulates GO:0045184 Sources: GOC:BHF, GOC:mah